{
  "term_label": "hexosaminidase activity",
  "gene_symbol": "OGA",
  "term_id": "GO:0015929",
  "gene": "UniProtKB:O60502",
  "gene_name": "Protein O-GlcNAcase"
}